{
  "gene_symbol": "RAB11FIP1",
  "term_label": "Unknown molecular function",
  "gene_name": "Rab11 family-interacting protein 1",
  "term_id": "UNKNOWN:0001",
  "gene": "UniProtKB:Q6WKZ4"
}